carbohydrate homeostasis [GO:0033500] (biological process) Subtypes: glucose homeostasis [GO:0042593] Relationships: is_a GO:0048878 Definition: A homeostatic process involved in the maintenance of an internal steady state of a carbohydrate within an organism or cell. Sources: GOC:mah